{
  "gene": "UniProtKB:Q5TB30",
  "gene_name": "DEP domain-containing protein 1A",
  "gene_symbol": "DEPDC1",
  "term_id": "UNKNOWN:0002",
  "term_label": "Unknown biological process"
}